peripheral B cell tolerance induction [GO:0002451] (biological process) Also known as: peripheral B lymphocyte tolerance induction, peripheral B-cell tolerance induction, peripheral B-lymphocyte tolerance induction Sources: GOC:jal, ISBN:0781735149 Subtypes: GO:0002402 Relationships: is a type of peripheral tolerance induction [GO:0002465]; is a type of B cell tolerance induction [GO:0002514]; is a type of B cell mediated immunity [GO:0019724] Definition: Tolerance induction of mature B cells in the peripheral lymphoid tissues: the blood, lymph nodes, spleen, and mucosal-associated lymphoid tissue.